{
  "gene_symbol": "LZTS1",
  "term_id": "GO:0043197",
  "gene_name": "Leucine zipper putative tumor suppressor 1",
  "term_label": "dendritic spine",
  "gene": "UniProtKB:Q9Y250"
}